pseudohyphal growth [GO:0007124] (BP) Definition: The process in which cells grow as a chain of physically attached, elongated cells in response to an environmental stimulus or stimuli. Relationships: is a type of GO:0016049; is a type of GO:0070783 References: PMID:11104818, PMID:19347739, PMID:24710476 Sources: GOC:krc Regulation: RO_0002211 by GO:2000220; negatively regulated by GO:2000221; RO_0002213 by GO:2000222